positive regulation of methane biosynthetic process from formic acid [GO:1900341] (biological process) Definition: Any process that activates or increases the frequency, rate or extent of methane biosynthetic process from formic acid. Also known as: up regulation of methane biosynthetic process from formic acid, up-regulation of methane biosynthetic process from formic acid, upregulation of methane biosynthetic process from formic acid, activation of methane biosynthetic process from formic acid Relationships: is a type of GO:0062013; is a type of regulation of methane biosynthetic process from formic acid [GO:1900339]; is a type of positive regulation of alkane biosynthetic process [GO:1901579]; is a type of positive regulation of cellular respiration [GO:1901857]; positively regulates methane biosynthetic process from formic acid [GO:2001127] Sources: GOC:TermGenie, GOC:mengo_curators